histone H4R3 methyltransferase activity [GO:0044020] (molecular function) Relationships: is a type of protein-arginine N-methyltransferase activity [GO:0016274]; is a type of GO:0140939 Definition: Catalysis of the reaction: S-adenosyl-L-methionine + (histone H4)-arginine (position 3) = S-adenosyl-L-homocysteine + (histone H4)-N-methyl-arginine (position 3). This reaction is the addition of a methyl group to the arginine residue at position 3 of histone H4, producing histone H4R3me. Note: Note that the residue position corresponds to the canonical human H4 histone (UniProtKB:P02309); this residue is conserved across all eukaryotes. Note that the initiation methionine is cleaved, so the first residue is S1. References: PMID:17898714 Sources: GOC:mah Also known as: histone H4KR3 methylation, histone H4R3 arginine methylase activity, histone methylase activity (H4-R3 specific), histone methyltransferase activity (H4-R3 specific), histone-arginine N-methyltransferase activity (H4-R3 specific)